phenylacetaldehyde reductase activity [GO:0102386] (molecular function) References: PMID:17644147 Sources: RHEA:63736 Definition: Catalysis of the reaction: 2-phenylacetaldehyde + NADPH + H+ = 2-phenylethanol + NADP+. Relationships: is a type of oxidoreductase activity, acting on the CH-OH group of donors, NAD or NADP as acceptor [GO:0016616]